{
  "term_id": "GO:0006325",
  "gene_symbol": "H2BW2",
  "gene": "UniProtKB:P0C1H6",
  "term_label": "chromatin organization",
  "gene_name": "Histone H2B type F-M"
}